dense core granule localization [GO:0032253] (biological process) Relationships: is a type of secretory granule localization [GO:0032252] Subtypes: dense core granule transport [GO:1901950], dense core granule exocytosis [GO:1990504] Also known as: dense core granule localisation, dense core vesicle localization, dense core granule clustering Definition: Any process in which a dense core granule is transported to, and/or maintained in, a specific location within the cell. Sources: GOC:mah